{
  "term_label": "cytokine-mediated signaling pathway",
  "gene_name": "Suppressor of cytokine signaling 5",
  "gene": "UniProtKB:O75159",
  "gene_symbol": "SOCS5",
  "term_id": "GO:0019221"
}